diphosphate-serine phosphotransferase activity [GO:0047332] (molecular function) Definition: Catalysis of the reaction: L-serine + diphosphate = O-phospho-L-serine + H+ + phosphate. Sources: EC:2.7.1.80, RHEA:23764 Also known as: diphosphate:L-serine O-phosphotransferase activity, pyrophosphate--serine phosphotransferase activity, pyrophosphate-L-serine phosphotransferase activity Relationships: is_a kinase activity [GO:0016301]; is_a GO:0016773